{
  "term_id": "GO:0098970",
  "gene": "UniProtKB:O60359",
  "gene_name": "Voltage-dependent calcium channel gamma-3 subunit",
  "term_label": "postsynaptic neurotransmitter receptor diffusion trapping",
  "gene_symbol": "CACNG3"
}